{
  "gene": "UniProtKB:P06307",
  "term_id": "GO:0005184",
  "gene_name": "Cholecystokinin",
  "term_label": "neuropeptide hormone activity",
  "gene_symbol": "CCK"
}